{
  "gene": "UniProtKB:Q9P2F9",
  "gene_name": "Zinc finger protein 319",
  "term_label": "nucleus",
  "gene_symbol": "ZNF319",
  "term_id": "GO:0005634"
}